UDP-N-acetylglucosamine transmembrane transport [GO:1990569] (biological process) Relationships: is a type of organic anion transport [GO:0015711]; is a type of GO:0090481 Also known as: UDP-N-acetylglucosamine transport References: PMID:10788474 Definition: The process in which UDP-N-acetylglucosamine is transported across a membrane.